negative regulation of Wnt protein secretion [GO:0061358] (biological process) Definition: Any process that stops, prevents, or reduces the frequency, rate or extent of the controlled release of a Wnt protein from a cell. References: PMID:19223472 Sources: GOC:bf Relationships: is a type of GO:0010648; is a type of negative regulation of signaling [GO:0023057]; is a type of negative regulation of protein secretion [GO:0050709]; is a type of GO:0061356; negatively regulates GO:0061355